{
  "gene": "UniProtKB:P01375",
  "term_label": "tumor necrosis factor-mediated signaling pathway",
  "term_id": "GO:0033209",
  "gene_name": "Tumor necrosis factor",
  "gene_symbol": "TNF"
}